{
  "gene_symbol": "ANKRD22",
  "gene": "UniProtKB:Q5VYY1",
  "term_label": "Unknown biological process",
  "gene_name": "Ankyrin repeat domain-containing protein 22",
  "term_id": "UNKNOWN:0002"
}